{
  "gene": "UniProtKB:P51800",
  "term_label": "plasma membrane",
  "term_id": "GO:0005886",
  "gene_symbol": "CLCNKA",
  "gene_name": "Chloride channel protein ClC-Ka"
}